{
  "gene_name": "Rho GTPase-activating protein 15",
  "gene": "UniProtKB:Q53QZ3",
  "term_id": "GO:0007264",
  "term_label": "small GTPase-mediated signal transduction",
  "gene_symbol": "ARHGAP15"
}